{
  "gene_name": "TBCC domain-containing protein 1",
  "gene_symbol": "TBCCD1",
  "term_label": "maintenance of Golgi location",
  "term_id": "GO:0051684",
  "gene": "UniProtKB:Q9NVR7"
}